{
  "gene_symbol": "SLFN12L",
  "gene": "UniProtKB:Q6IEE8",
  "term_label": "Unknown cellular component",
  "term_id": "UNKNOWN:0003",
  "gene_name": "Schlafen family member 12-like"
}